{
  "term_id": "UNKNOWN:0003",
  "gene": "UniProtKB:C0HLZ6",
  "term_label": "Unknown cellular component",
  "gene_name": "HOXB-AS3 peptide",
  "gene_symbol": "HOXB-AS3"
}